{
  "term_id": "GO:0005654",
  "gene_symbol": "NKRF",
  "term_label": "nucleoplasm",
  "gene_name": "NF-kappa-B-repressing factor",
  "gene": "UniProtKB:O15226"
}